transcription antitermination [GO:0031564] (biological process) References: PMID:12456320, PMID:21478900, PMID:30191803 Sources: ISBN:0198577788 Also known as: transcriptional readthrough Definition: A positive regulation of gene expression mechanism that allows RNA polymerase to continue transcription beyond a termination site, thus allowing expression of downstream genes under specific conditions. Relationships: is a type of GO:0010628; is a type of negative regulation of termination of DNA-templated transcription [GO:0060567]